2,4,6-trinitrotoluene catabolic process [GO:0046256] (biological process) Relationships: is a type of trinitrotoluene catabolic process [GO:0046260] Subtypes: anaerobic 2,4,6-trinitrotoluene catabolic process [GO:0046258] Sources: GOC:ai Definition: The chemical reactions and pathways resulting in the breakdown of 2,4,6-trinitrotoluene, 1-methyl-2,4,6-trinitrobenzene, a highly explosive pale yellow crystalline solid. Also known as: 2,4,6-trinitrotoluene breakdown, 2,4,6-trinitrotoluene catabolism, 2,4,6-trinitrotoluene degradation